{
  "gene": "UniProtKB:Q7L5Y6",
  "gene_symbol": "DET1",
  "term_label": "protein ubiquitination",
  "gene_name": "DET1 homolog",
  "term_id": "GO:0016567"
}